gonad development [GO:0008406] (biological process) Definition: The process whose specific outcome is the progression of the gonad over time, from its formation to the mature structure. The gonad is an animal organ that produces gametes; in some species it also produces hormones. Relationships: is a type of animal organ development [GO:0048513]; is a type of reproductive structure development [GO:0048608]; is part of development of primary sexual characteristics [GO:0045137] Sources: GOC:ems, ISBN:0198506732 Also known as: gonadogenesis Subtypes: GO:0008584, GO:0008585 Regulation: regulated by GO:1905939; negatively regulated by negative regulation of gonad development [GO:1905940]; positively regulated by positive regulation of gonad development [GO:1905941]